{
  "term_label": "cAMP-dependent protein kinase complex",
  "gene_symbol": "PRKACA",
  "gene_name": "cAMP-dependent protein kinase catalytic subunit alpha",
  "gene": "UniProtKB:P17612",
  "term_id": "GO:0005952"
}